{
  "gene_name": "Serine_threonine-protein kinase PDIK1L",
  "term_id": "GO:0005737",
  "gene_symbol": "PDIK1L",
  "gene": "UniProtKB:Q8N165",
  "term_label": "cytoplasm"
}